{
  "gene": "UniProtKB:P10645",
  "term_label": "extracellular space",
  "term_id": "GO:0005615",
  "gene_symbol": "CHGA",
  "gene_name": "Chromogranin-A"
}